crotonobetaine-CoA ligase activity [GO:0051109] (molecular function) Relationships: is a type of GO:0016405 Sources: MetaCyc:CROTCOALIG-RXN Definition: Catalysis of the reaction: CoA + crotono-betaine + ATP = AMP + diphosphate + crotonobetainyl-CoA. Also known as: crotonobetaine/carnitine-CoA ligase activity, crotonobetaine-CoA synthase activity